{
  "gene_symbol": "TP53BP1",
  "gene_name": "TP53-binding protein 1",
  "term_label": "nucleus",
  "gene": "UniProtKB:Q12888",
  "term_id": "GO:0005634"
}